{
  "gene_name": "Probable 28S rRNA (cytosine(4447)-C(5))-methyltransferase",
  "gene_symbol": "NOP2",
  "gene": "UniProtKB:P46087",
  "term_label": "maturation of LSU-rRNA",
  "term_id": "GO:0000470"
}